immunological memory process [GO:0090713] (biological process) Definition: Any process of the immune system that can contribute to the formation of immunological memory or an immune response based upon activation of immunological memory. References: PMID:26086132, PMID:26831526 Sources: GOC:add Relationships: is a type of immune system process [GO:0002376]; is part of immune response [GO:0006955] Subtypes: innate immunity memory response [GO:0090714], immunological memory formation process [GO:0090715], adaptive immune memory response [GO:0090716]